{
  "gene_name": "Heat shock factor protein 1",
  "gene_symbol": "HSF1",
  "term_label": "RNA polymerase II cis-regulatory region sequence-specific DNA binding",
  "term_id": "GO:0000978",
  "gene": "UniProtKB:Q00613"
}